{
  "term_id": "GO:0030133",
  "gene_name": "Ankyrin repeat domain-containing protein 27",
  "term_label": "transport vesicle",
  "gene_symbol": "ANKRD27",
  "gene": "UniProtKB:Q96NW4"
}